{
  "gene_symbol": "NOL4L",
  "gene_name": "Nucleolar protein 4-like",
  "term_label": "Unknown biological process",
  "term_id": "UNKNOWN:0002",
  "gene": "UniProtKB:Q96MY1"
}